{
  "term_id": "GO:0043315",
  "term_label": "positive regulation of neutrophil degranulation",
  "gene": "UniProtKB:Q8N6Q3",
  "gene_symbol": "CD177",
  "gene_name": "CD177 antigen"
}